{
  "gene_symbol": "SP5",
  "term_label": "nucleus",
  "gene_name": "Transcription factor Sp5",
  "gene": "UniProtKB:Q6BEB4",
  "term_id": "GO:0005634"
}